{
  "term_id": "GO:0042391",
  "gene": "UniProtKB:Q8NE79",
  "term_label": "regulation of membrane potential",
  "gene_name": "Blood vessel epicardial substance",
  "gene_symbol": "BVES"
}